{
  "gene_symbol": "OR14L1",
  "gene_name": "Olfactory receptor 14L1",
  "term_label": "Unknown biological process",
  "term_id": "UNKNOWN:0002",
  "gene": "UniProtKB:Q8NHC6"
}